cyclic pyranopterin monophosphate synthase activity [GO:0061799] (molecular function) Definition: Catalysis of the reaction: (8S)-3',8-cyclo-7,8-dihydroguanosine 5'-triphosphate = cyclic pyranopterin phosphate + diphosphate. References: PMID:25896388 Sources: GOC:dph, GOC:ik Relationships: is a type of GO:0016849